retrograde trans-synaptic signaling by lipid [GO:0098920] (biological process) Sources: GOC:dos Subtypes: retrograde trans-synaptic signaling by endocannabinoid [GO:0098921] Relationships: is a type of retrograde trans-synaptic signaling [GO:0098917]; is a type of GO:0099541 Definition: Cell-cell signaling from postsynapse to presynapse, across the synaptic cleft, mediated by a lipid ligand.